renal filtration [GO:0097205] (biological process) Definition: A renal system process in which fluid circulating through the body is filtered through a barrier system. Relationships: is a type of GO:0003014 Sources: GOC:pr, GOC:sart Subtypes: glomerular filtration [GO:0003094], nephrocyte filtration [GO:0097206]